{
  "gene_name": "Homeobox protein Hox-C9",
  "term_id": "GO:0005634",
  "term_label": "nucleus",
  "gene": "UniProtKB:P31274",
  "gene_symbol": "HOXC9"
}